{
  "gene_name": "Calcium uptake protein 2, mitochondrial",
  "term_id": "GO:0051560",
  "term_label": "mitochondrial calcium ion homeostasis",
  "gene_symbol": "MICU2",
  "gene": "UniProtKB:Q8IYU8"
}